{
  "term_label": "lamellipodium",
  "gene_name": "Unconventional myosin-IXb",
  "gene": "UniProtKB:Q13459",
  "term_id": "GO:0030027",
  "gene_symbol": "MYO9B"
}